{
  "gene": "UniProtKB:P07225",
  "gene_symbol": "PROS1",
  "gene_name": "Vitamin K-dependent protein S",
  "term_id": "GO:0005615",
  "term_label": "extracellular space"
}